{
  "gene_symbol": "SNRPD2",
  "term_label": "precatalytic spliceosome",
  "gene": "UniProtKB:P62316",
  "term_id": "GO:0071011",
  "gene_name": "Small nuclear ribonucleoprotein Sm D2"
}